{
  "gene": "UniProtKB:Q8TC36",
  "gene_symbol": "SUN5",
  "term_id": "GO:0005635",
  "gene_name": "SUN domain-containing protein 5",
  "term_label": "nuclear envelope"
}